{
  "term_id": "GO:0030425",
  "gene_symbol": "KIF1A",
  "gene_name": "Kinesin-like protein KIF1A",
  "gene": "UniProtKB:Q12756",
  "term_label": "dendrite"
}